{
  "gene_symbol": "ARID1B",
  "gene": "UniProtKB:Q8NFD5",
  "term_label": "nucleosome binding",
  "gene_name": "AT-rich interactive domain-containing protein 1B",
  "term_id": "GO:0031491"
}